{
  "gene_symbol": "OR52K1",
  "term_label": "Unknown biological process",
  "gene": "UniProtKB:Q8NGK4",
  "gene_name": "Olfactory receptor 52K1",
  "term_id": "UNKNOWN:0002"
}